thrombin-activated receptor signaling pathway [GO:0070493] (BP) Also known as: thrombin receptor signaling pathway, thrombin receptor signalling pathway References: PMID:1672265 Sources: GOC:mah Relationships: is a type of G protein-coupled receptor signaling pathway [GO:0007186] Regulation: regulated by GO:0070494; negatively regulated by negative regulation of thrombin-activated receptor signaling pathway [GO:0070495]; positively regulated by GO:0070496 Definition: A G protein-coupled receptor signaling pathway initiated by thrombin binding to its receptor on the surface of a target cell, and ending with the regulation of a downstream cellular process.